{
  "gene": "UniProtKB:Q9H4B7",
  "gene_symbol": "TUBB1",
  "term_id": "GO:0000226",
  "term_label": "microtubule cytoskeleton organization",
  "gene_name": "Tubulin beta-1 chain"
}